{
  "gene_name": "Putative PRAME family member 13",
  "term_id": "GO:0005737",
  "term_label": "cytoplasm",
  "gene": "UniProtKB:Q5VWM6",
  "gene_symbol": "PRAMEF13"
}